ferric-chelate reductase activity [GO:0000293] (molecular function) References: PMID:33559753 Relationships: is a type of oxidoreductase activity, acting on metal ions [GO:0016722] Also known as: ferric chelate reductase activity, iron chelate reductase activity Subtypes: GO:0052851, ferric-chelate reductase (NADH) activity [GO:0140618] Definition: Catalysis of the reaction: 2 Fe3+-siderophore + electron donor = 2 Fe2+-siderophore + electron acceptor.